metanephric proximal convoluted tubule segment 1 development [GO:0072231] (biological process) Definition: The process whose specific outcome is the progression of the S1 portion of the metanephric proximal convoluted tubule over time, from its formation to the mature structure. The S1 portion is the initial portion of the metanephric proximal convoluted tubule and is responsible for avid reabsorption of water and solutes. Sources: GOC:bf, GOC:mtg_kidney_jan10 Also known as: metanephric S1 development Relationships: is a type of proximal convoluted tubule segment 1 development [GO:0072031]; is part of metanephric proximal convoluted tubule development [GO:0072229]